{
  "gene_symbol": "RPLP0P6",
  "term_id": "GO:0002181",
  "gene_name": "Putative ribosomal protein uL10-like",
  "term_label": "cytoplasmic translation",
  "gene": "UniProtKB:Q8NHW5"
}